pedicel mucilage biosynthetic process [GO:0048357] (biological process) Also known as: pedicel mucilage anabolism, pedicel mucilage biosynthesis, pedicel mucilage formation, pedicel mucilage synthesis Sources: GOC:jid Definition: The chemical reactions and pathways resulting in the formation of mucilage that occur in the flower stem. Relationships: is a type of mucilage biosynthetic process [GO:0010192]